{
  "term_label": "Unknown biological process",
  "gene": "UniProtKB:A8MUN3",
  "term_id": "UNKNOWN:0002",
  "gene_name": "Putative uncharacterized protein ENSP00000381830",
  "gene_symbol": "A8MUN3"
}